cellularization cleavage furrow invagination front [GO:0110071] (cellular component) Relationships: is a type of cellular anatomical structure [GO:0110165]; is part of cellularization cleavage furrow [GO:0110070] Definition: The base of the cellularization invagination or cleavage furrow most distal to the original multi-nucleate cell or syncytium plasma membrane. References: PMID:27226317 Sources: GOC:ha